{
  "gene": "UniProtKB:P62072",
  "term_label": "membrane insertase activity",
  "gene_symbol": "TIMM10",
  "term_id": "GO:0032977",
  "gene_name": "Mitochondrial import inner membrane translocase subunit Tim10"
}